{
  "gene": "UniProtKB:Q9UBG3",
  "gene_name": "Cornulin",
  "term_id": "GO:0048306",
  "gene_symbol": "CRNN",
  "term_label": "calcium-dependent protein binding"
}